response to dexamethasone [GO:0071548] (biological process) Definition: Any process that results in a change in state or activity of a cell or an organism (in terms of movement, secretion, enzyme production, gene expression, etc.) as a result of a dexamethasone stimulus. Sources: GOC:mah, GOC:yaf Also known as: response to dexamethasone stimulus Relationships: is a type of response to glucocorticoid [GO:0051384]; is a type of response to ketone [GO:1901654] Subtypes: GO:0071549